hyperosmotic salinity response [GO:0042538] (biological process) Also known as: response to hyperosmotic salt stress, salt tolerance Relationships: is a type of hyperosmotic response [GO:0006972]; is a type of response to salt stress [GO:0009651] Definition: Any process that results in a change in state or activity of a cell or an organism (in terms of movement, secretion, enzyme production, gene expression, etc.) as a result of detection of, or exposure to, an increase in the concentration of salt (particularly but not exclusively sodium and chloride ions) in the environment. Sources: GOC:jl Subtypes: cellular hyperosmotic salinity response [GO:0071475]